{
  "term_id": "GO:0005737",
  "term_label": "cytoplasm",
  "gene": "UniProtKB:Q9BWT7",
  "gene_name": "Caspase recruitment domain-containing protein 10",
  "gene_symbol": "CARD10"
}